{
  "term_label": "Unknown biological process",
  "term_id": "UNKNOWN:0002",
  "gene_name": "GRAM domain-containing protein 2B",
  "gene": "UniProtKB:Q96HH9",
  "gene_symbol": "GRAMD2B"
}